positive regulation of AMPA glutamate receptor clustering [GO:1904719] (biological process) Also known as: positive regulation of AMPA receptor clustering, positive regulation of alpha-amino-3-hydroxy-5-methyl-4-isoxazole propionate selective glutamate receptor clustering, up regulation of AMPA glutamate receptor clustering, up regulation of AMPA receptor clustering, up regulation of alpha-amino-3-hydroxy-5-methyl-4-isoxazole propionate selective glutamate receptor clustering, up-regulation of AMPA glutamate receptor clustering, up-regulation of AMPA receptor clustering, up-regulation of alpha-amino-3-hydroxy-5-methyl-4-isoxazole propionate selective glutamate receptor clustering, upregulation of AMPA glutamate receptor clustering, upregulation of AMPA receptor clustering, upregulation of alpha-amino-3-hydroxy-5-methyl-4-isoxazole propionate selective glutamate receptor clustering, activation of AMPA glutamate receptor clustering, activation of AMPA receptor clustering, activation of alpha-amino-3-hydroxy-5-methyl-4-isoxazole propionate selective glutamate receptor clustering Definition: Any process that activates or increases the frequency, rate or extent of AMPA glutamate receptor clustering. References: PMID:21558424 Sources: GOC:TermGenie, GOC:hjd, GO_REF:0000058 Relationships: is a type of positive regulation of postsynaptic membrane organization [GO:1901628]; is a type of GO:1903911; is a type of regulation of AMPA glutamate receptor clustering [GO:1904717]; positively regulates AMPA glutamate receptor clustering [GO:0097113]